{
  "gene_symbol": "CCDC113",
  "term_label": "Unknown molecular function",
  "gene": "UniProtKB:Q9H0I3",
  "gene_name": "Coiled-coil domain-containing protein 113",
  "term_id": "UNKNOWN:0001"
}